tetrahydrofolate interconversion [GO:0035999] (biological process) Definition: The chemical reactions and pathways by which one-carbon (C1) units are transferred between tetrahydrofolate molecules, to synthesize other tetrahydrofolate molecules. References: PMID:1825999 Sources: GOC:yaf Relationships: is a type of one-carbon metabolic process [GO:0006730]; is_a GO:0046653